{
  "term_id": "GO:1901911",
  "gene": "UniProtKB:O95989",
  "gene_symbol": "NUDT3",
  "gene_name": "Diphosphoinositol polyphosphate phosphohydrolase 1",
  "term_label": "adenosine 5'-(hexahydrogen pentaphosphate) catabolic process"
}